{
  "term_id": "UNKNOWN:0002",
  "gene_symbol": "PRRT4",
  "gene": "UniProtKB:C9JH25",
  "term_label": "Unknown biological process",
  "gene_name": "Proline-rich transmembrane protein 4"
}